{
  "term_id": "GO:0005886",
  "term_label": "plasma membrane",
  "gene": "UniProtKB:O43511",
  "gene_name": "Pendrin",
  "gene_symbol": "SLC26A4"
}